{
  "gene_name": "Zinc finger protein 772",
  "gene": "UniProtKB:Q68DY9",
  "term_id": "GO:0006357",
  "term_label": "regulation of transcription by RNA polymerase II",
  "gene_symbol": "ZNF772"
}